phosphoenolpyruvate carboxykinase activity [GO:0004611] (MF) Subtypes: phosphoenolpyruvate carboxykinase (ATP) activity [GO:0004612], GO:0004613, GO:0008964, phosphoenolpyruvate carboxykinase (diphosphate) activity [GO:0030585] Sources: GOC:curators Definition: Catalysis of the reaction: phosphate + oxaloacetate = phosphoenolpyruvate + CO2 + other reaction products. Relationships: is a type of carboxy-lyase activity [GO:0016831] Also known as: PEP carboxykinase activity, PEPCK activity, phosphopyruvate carboxylase activity